ATP-dependent H3-H4 histone complex chaperone activity [GO:0140665] (molecular function) References: PMID:31848341, PMID:33658433 Definition: A histone chaperone that carries a H3-H4 histone complex, driven by ATP hydrolysis. Relationships: is a type of H3-H4 histone complex chaperone activity [GO:0000510]; is a type of GO:0140674 Also known as: H3-H4 histone chaperone, H3-H4 histone complex loader activity, H3-H4 dimer loading activity, histone H3-H4 dimer loading activity, ATP-dependent H3-H4 histone complex loader activity, histone chaperone